intracellular manganese ion homeostasis [GO:0030026] (biological process) Definition: A homeostatic process involved in the maintenance of a steady state level of manganese ions within a cell. Relationships: is a type of intracellular monoatomic cation homeostasis [GO:0030003]; is a type of manganese ion homeostasis [GO:0055071] Also known as: manganese homeostasis, cellular manganese ion homeostasis Sources: GOC:mah